{
  "gene": "UniProtKB:P08134",
  "term_label": "GTPase activity",
  "gene_symbol": "RHOC",
  "gene_name": "Rho-related GTP-binding protein RhoC",
  "term_id": "GO:0003924"
}